{
  "gene_symbol": "TTC21B",
  "term_label": "intraciliary retrograde transport",
  "gene_name": "Tetratricopeptide repeat protein 21B",
  "gene": "UniProtKB:Q7Z4L5",
  "term_id": "GO:0035721"
}